{
  "term_id": "GO:0007399",
  "gene_symbol": "SRGAP3",
  "gene": "UniProtKB:O43295",
  "term_label": "nervous system development",
  "gene_name": "SLIT-ROBO Rho GTPase-activating protein 3"
}